{
  "term_label": "axon",
  "gene_symbol": "CCSAP",
  "gene": "UniProtKB:Q6IQ19",
  "gene_name": "Centriole, cilia and spindle-associated protein",
  "term_id": "GO:0030424"
}